small RNA binding translational repressor activity [GO:0140764] (MF) Note: This term is intended for activities such as that mediated by argonaute in the RISC complex, that bring a miRNA or an siRNA to their target mRNA. Definition: A translational repressor activity that binds to a single-stranded small regulatory RNA (either a miRNA or a siRNA) to guide it to its target mRNA. References: PMID:27184117, PMID:34117606 Relationships: is a type of GO:0030371; is part of post-transcriptional gene silencing [GO:0016441]; has part GO:0061980